{
  "gene": "UniProtKB:Q711Q0",
  "term_id": "GO:0070886",
  "term_label": "positive regulation of calcineurin-NFAT signaling cascade",
  "gene_name": "Cardiac-enriched FHL2-interacting protein",
  "gene_symbol": "CEFIP"
}